{
  "gene": "UniProtKB:A0A0A0MS05",
  "gene_name": "Probable non-functional T cell receptor beta variable 5-7",
  "gene_symbol": "TRBV5-7",
  "term_label": "plasma membrane",
  "term_id": "GO:0005886"
}